{
  "gene_name": "Collectin-10",
  "term_label": "extracellular space",
  "gene_symbol": "COLEC10",
  "gene": "UniProtKB:Q9Y6Z7",
  "term_id": "GO:0005615"
}